{
  "gene": "UniProtKB:Q6ZS52",
  "gene_symbol": "Q6ZS52",
  "term_label": "Unknown biological process",
  "term_id": "UNKNOWN:0002",
  "gene_name": "Putative uncharacterized protein FLJ45825"
}